D-pinitol dehydrogenase activity [GO:0047832] (molecular function) Sources: EC:1.1.1.142, RHEA:20437 Also known as: 1D-3-O-methyl-chiro-inositol:NADP+ oxidoreductase activity, 5D-5-O-methyl-chiro-inositol:NADP+ oxidoreductase activity Definition: Catalysis of the reaction: 5D-5-O-methyl-chiro-inositol + NADP+ = 2D-5-O-methyl-2,3,5/4,6-pentahydroxycyclohexanone + H+ + NADPH. Relationships: is a type of oxidoreductase activity, acting on the CH-OH group of donors, NAD or NADP as acceptor [GO:0016616]